regulation of cytokine-mediated signaling pathway [GO:0001959] (BP) Also known as: regulation of cytokine and chemokine mediated signaling pathway, regulation of cytokine mediated signaling pathway, regulation of cytokine mediated signalling pathway Sources: GOC:hjd Definition: Any process that modulates the frequency, rate or extent of the cytokine mediated signaling pathway. Subtypes: negative regulation of cytokine-mediated signaling pathway [GO:0001960], positive regulation of cytokine-mediated signaling pathway [GO:0001961], regulation of tumor necrosis factor-mediated signaling pathway [GO:0010803], regulation of type II interferon-mediated signaling pathway [GO:0060334], GO:0060338, regulation of chemokine-mediated signaling pathway [GO:0070099], regulation of interleukin-6-mediated signaling pathway [GO:0070103], GO:0070107, regulation of interleukin-35-mediated signaling pathway [GO:0070758], regulation of Kit signaling pathway [GO:1900234], regulation of interleukin-2-mediated signaling pathway [GO:1902205], regulation of prolactin signaling pathway [GO:1902211], regulation of interleukin-4-mediated signaling pathway [GO:1902214], regulation of macrophage colony-stimulating factor signaling pathway [GO:1902226], GO:1903881, GO:2000446, regulation of interleukin-18-mediated signaling pathway [GO:2000492], regulation of interleukin-1-mediated signaling pathway [GO:2000659] Relationships: is a type of GO:0009966; is a type of GO:0060759; regulates cytokine-mediated signaling pathway [GO:0019221]